{
  "term_label": "Unknown biological process",
  "gene_symbol": "FAM72B",
  "term_id": "UNKNOWN:0002",
  "gene": "UniProtKB:Q86X60",
  "gene_name": "Protein FAM72B"
}